{
  "term_id": "GO:0000146",
  "gene_name": "Unconventional myosin-XIX",
  "gene_symbol": "MYO19",
  "term_label": "microfilament motor activity",
  "gene": "UniProtKB:Q96H55"
}